{
  "gene_name": "E3 ubiquitin-protein ligase Arkadia",
  "term_id": "GO:0005634",
  "term_label": "nucleus",
  "gene_symbol": "RNF111",
  "gene": "UniProtKB:Q6ZNA4"
}